regulation of vasoconstriction [GO:0019229] (biological process) Sources: GOC:jl Relationships: is a type of blood vessel diameter maintenance [GO:0097746]; is a type of regulation of blood circulation [GO:1903522]; regulates GO:0042310 Definition: Any process that modulates the frequency, rate or extent of reductions in the diameter of blood vessels. Subtypes: regulation of vascular associated smooth muscle contraction [GO:0003056], regulation of vasoconstriction by epinephrine [GO:0003115], regulation of vasoconstriction by norepinephrine [GO:0003116], negative regulation of vasoconstriction [GO:0045906], positive regulation of vasoconstriction [GO:0045907]